{
  "gene_symbol": "OR8G1",
  "term_id": "UNKNOWN:0003",
  "gene_name": "Olfactory receptor 8G1",
  "gene": "UniProtKB:Q15617",
  "term_label": "Unknown cellular component"
}